glutathione import into mitochondrion [GO:0160007] (biological process) Relationships: is a type of glutathione transmembrane transport [GO:0034775] Definition: The process in which glutathione is transported from the cytosol into the mitochondrial matrix. References: PMID:34707288